{
  "gene": "UniProtKB:Q8IWQ3",
  "term_id": "GO:0007409",
  "gene_symbol": "BRSK2",
  "term_label": "axonogenesis",
  "gene_name": "Serine_threonine-protein kinase BRSK2"
}